epidermal cell differentiation [GO:0009913] (biological process) Also known as: hypodermal cell differentiation Sources: GOC:dph, GOC:go_curators, GOC:mtg_sensu, GOC:sdb_2009, GOC:tb Subtypes: GO:0001949, GO:0030216, hair cell differentiation [GO:0035315], GO:0060889 Regulation: regulated by regulation of epidermal cell differentiation [GO:0045604]; negatively regulated by negative regulation of epidermal cell differentiation [GO:0045605]; positively regulated by positive regulation of epidermal cell differentiation [GO:0045606] Relationships: is a type of epithelial cell differentiation [GO:0030855]; is part of epidermis development [GO:0008544] Definition: The process in which a relatively unspecialized cell acquires specialized features of an epidermal cell, any of the cells making up the epidermis.